{
  "gene": "UniProtKB:A2VDF0",
  "gene_symbol": "FUOM",
  "term_id": "GO:0042806",
  "gene_name": "Fucose mutarotase",
  "term_label": "fucose binding"
}